glutathione synthase complex [GO:0036087] (cellular component) Relationships: is a type of GO:1902494 Definition: A protein complex composed of two or more polypeptide subunits, and which possesses glutathione synthase activity (catalysis of the reaction: L-gamma-glutamyl-L-cysteine + ATP + glycine = ADP + glutathione + 2 H+ + phosphate). In eukaryotes, the complex is homodimeric, in E. coli glutathione synthase exists as a tetramer, and in S. pombe the complex exists as a homodimer or a heterotetramer. Also known as: glutathione synthetase complex References: PMID:12734194, PMID:14990577, PMID:1958212 Sources: GOC:al